positive regulation by symbiont of entry into host [GO:0075294] (biological process) Relationships: is a type of positive regulation of biological process [GO:0048518]; is_a GO:0052372; positively regulates symbiont entry into host [GO:0044409] Definition: Any process that activates or increases the frequency, rate or extent to which it enters into the host organism, where the two organisms are in a symbiotic interaction. Also known as: up regulation by symbiont of entry into host, up-regulation by symbiont of entry into host, upregulation by symbiont of entry into host, activation by organism of entry into other organism during symbiotic interaction, activation by symbiont of entry into host, positive regulation by organism of entry into other organism during symbiotic interaction, positive regulation by organism of entry into other organism involved in symbiotic interaction, up regulation by organism of entry into other organism during symbiotic interaction, up-regulation by organism of entry into other organism during symbiotic interaction, upregulation by organism of entry into other organism during symbiotic interaction Subtypes: positive regulation of viral entry into host cell [GO:0046598], GO:0075055, positive regulation of symbiont haustorium neck formation for entry into host [GO:0075199], positive regulation of penetration hypha formation [GO:0075203] Sources: GOC:pamgo_curators